L-arabinofuranose binding [GO:2001084] (molecular function) Definition: Binding to L-arabinofuranose. Sources: GOC:mengo_curators Relationships: is a type of monosaccharide binding [GO:0048029]